ATPase regulator activity [GO:0060590] (molecular function) Definition: Binds to and modulates the activity of an ATP hydrolysis activity. Also known as: ATP hydrolysis regulator activity Sources: GOC:dph, GOC:tb Relationships: is a type of molecular function regulator activity [GO:0098772]; regulates ATP-dependent activity [GO:0140657] Subtypes: adenyl-nucleotide exchange factor activity [GO:0000774], ATPase activator activity [GO:0001671], ATPase inhibitor activity [GO:0042030], DNA topoisomerase type II (double strand cut, ATP-hydrolyzing) regulator activity [GO:0072586]